{
  "gene": "UniProtKB:P30926",
  "term_id": "GO:0005892",
  "gene_symbol": "CHRNB4",
  "gene_name": "Neuronal acetylcholine receptor subunit beta-4",
  "term_label": "acetylcholine-gated channel complex"
}